microcin transmembrane transporter activity [GO:0015638] (molecular function) Also known as: microcin uptake permease activity Sources: GOC:mah Definition: Enables the transfer of a microcin from one side of a membrane to the other. Relationships: is a type of amide transmembrane transporter activity [GO:0042887]; is a type of xenobiotic transmembrane transporter activity [GO:0042910]; is part of microcin transport [GO:0042884]